{
  "gene": "UniProtKB:P07311",
  "gene_symbol": "ACYP1",
  "gene_name": "Acylphosphatase-1",
  "term_id": "UNKNOWN:0002",
  "term_label": "Unknown biological process"
}